protoxylem development [GO:0090059] (biological process) Relationships: is a type of xylem development [GO:0010089] Definition: The process whose specific outcome is the progression of the protoxylem over time, from its formation to the mature structure. The protoxylem comprises the first formed elements of the primary xylem. Sources: GOC:dph, GOC:sdb_2009, GOC:tb